T cell mediated cytotoxicity directed against tumor cell target [GO:0002419] (biological process) Relationships: is a type of T cell mediated cytotoxicity [GO:0001913]; is a type of T cell mediated immune response to tumor cell [GO:0002424] Also known as: T lymphocyte mediated cytotoxicity directed against tumor cell target, T-cell mediated cytotoxicity directed against tumor cell target, T-lymphocyte mediated cytotoxicity directed against tumor cell target Note: Note that either or both mechanisms mentioned in the definition may be used in this process. Note that both granule release and the engagement of death receptors on target cells result in induction of apoptosis in the target cell. References: PMID:16730260 Sources: GOC:add, ISBN:0781735149 Definition: The directed killing of a tumor cell by a T cell through the release of granules containing cytotoxic mediators or through the engagement of death receptors. Regulation: regulated by regulation of T cell mediated cytotoxicity directed against tumor cell target [GO:0002852]; RO_0002212 by negative regulation of T cell mediated cytotoxicity directed against tumor cell target [GO:0002853]; positively regulated by positive regulation of T cell mediated cytotoxicity directed against tumor cell target [GO:0002854]